adrenomedullin receptor complex [GO:1903143] (cellular component) References: PMID:22102369 Sources: GOC:TermGenie, GOC:bhm, GO_REF:0000088 Note: An example of this is RAMP2 in human (O60895) in PMID:22102369 (inferred from direct assay). Relationships: is a type of GO:0038037; is a type of calcitonin family receptor complex [GO:1903439] Definition: A transmembrane, G protein-coupled signaling receptor complex which is capable of adrenomedullin receptor activity. Also known as: adrenomedullin receptor AM1 complex, adrenomedullin receptor AM2 complex